viral DNA genome packaging, 5' extended cos packaging [GO:0098037] (biological process) Sources: GOC:bm Definition: The encapsulation of the viral DNA genome within the capsid, which proceeds via cleavage of the viral DNA at specific sites to produce 5' protruding ends. Relationships: is a type of viral DNA genome packaging via site-specific sequence recognition [GO:0098035]